{
  "gene_name": "Putative uncharacterized protein PRO0461",
  "gene_symbol": "PRO0461",
  "gene": "UniProtKB:Q9UI25",
  "term_id": "UNKNOWN:0001",
  "term_label": "Unknown molecular function"
}